{
  "term_id": "UNKNOWN:0001",
  "gene_symbol": "PATE3",
  "term_label": "Unknown molecular function",
  "gene_name": "Prostate and testis expressed protein 3",
  "gene": "UniProtKB:B3GLJ2"
}